{
  "gene": "UniProtKB:Q9BWF2",
  "gene_symbol": "TRAIP",
  "term_label": "replication fork processing",
  "term_id": "GO:0031297",
  "gene_name": "E3 ubiquitin-protein ligase TRAIP"
}